{
  "gene_name": "Histone-lysine N-methyltransferase KMT5C",
  "gene_symbol": "KMT5C",
  "term_label": "Unknown biological process",
  "gene": "UniProtKB:Q86Y97",
  "term_id": "UNKNOWN:0002"
}